{
  "term_label": "plasma membrane",
  "gene": "UniProtKB:Q8NGS8",
  "term_id": "GO:0005886",
  "gene_symbol": "OR13C5",
  "gene_name": "Olfactory receptor 13C5"
}